{
  "gene": "UniProtKB:Q9BRV8",
  "term_id": "UNKNOWN:0003",
  "gene_name": "Suppressor of IKBKE 1",
  "gene_symbol": "SIKE1",
  "term_label": "Unknown cellular component"
}